{
  "term_label": "mitochondrial membrane",
  "gene_name": "Interferon alpha-inducible protein 27, mitochondrial",
  "gene_symbol": "IFI27",
  "gene": "UniProtKB:P40305",
  "term_id": "GO:0031966"
}